{
  "gene_symbol": "REG3G",
  "term_id": "GO:0008083",
  "gene": "UniProtKB:Q6UW15",
  "term_label": "growth factor activity",
  "gene_name": "Regenerating islet-derived protein 3-gamma"
}